heart valve morphogenesis [GO:0003179] (biological process) Sources: GOC:mtg_heart Relationships: is_a anatomical structure morphogenesis [GO:0009653]; BFO_0000050 heart valve development [GO:0003170] Subtypes: GO:0003180, GO:0003181, coronary sinus valve morphogenesis [GO:0003182], GO:0003184, GO:0003185, GO:0003187 Also known as: heart valve remodeling, heart valve remodelling Definition: The process in which the structure of a heart valve is generated and organized.